N-benzyloxycarbonylglycine hydrolase activity [GO:0050125] (molecular function) Sources: EC:3.5.1.58, RHEA:20900 Definition: Catalysis of the reaction: N-benzyloxycarbonylglycine + H2O + H+ = benzyl alcohol + CO2 + glycine. Relationships: is a type of hydrolase activity, acting on carbon-nitrogen (but not peptide) bonds, in linear amides [GO:0016811] Also known as: N-benzyloxycarbonylglycine urethanehydrolase activity, benzyloxycarbonylglycine hydrolase activity, nalpha-benzyloxycarbonyl amino acid urethane hydrolase I, nalpha-benzyloxycarbonyl amino acid urethane hydrolase activity, nalpha-carbobenzoxyamino acid amidohydrolase activity